positive regulation of bone resorption [GO:0045780] (biological process) Sources: GOC:go_curators Also known as: up regulation of bone resorption, up-regulation of bone resorption, upregulation of bone resorption, activation of bone resorption, stimulation of bone resorption Relationships: is a type of GO:0045124; is_a GO:0051240; positively regulates bone resorption [GO:0045453] Definition: Any process that activates or increases the frequency, rate or extent of bone resorption.